regulation of catabolic process [GO:0009894] (biological process) Also known as: regulation of breakdown, regulation of catabolism, regulation of degradation Definition: Any process that modulates the frequency, rate, or extent of the chemical reactions and pathways resulting in the breakdown of substances. Sources: GOC:go_curators Subtypes: regulation of mitochondrial RNA catabolic process [GO:0000960], GO:0009895, positive regulation of catabolic process [GO:0009896], regulation of autophagy [GO:0010506], GO:0010567, GO:0010710, GO:0030811, regulation of amine catabolic process [GO:0033241], regulation of penicillin catabolic process [GO:0033247], regulation of amide catabolic process [GO:0034251], GO:0042176, regulation of carbohydrate catabolic process [GO:0043470], regulation of RNA stability [GO:0043487], regulation of acetate catabolic process [GO:0045734], GO:0050994, regulation of mRNA catabolic process [GO:0061013], regulation protein catabolic process at synapse [GO:0140250], regulation of anthocyanin catabolic process [GO:1900000], regulation of coenzyme F420-dependent bicyclic nitroimidazole catabolic process [GO:1900288], regulation of alcohol catabolic process [GO:1900419], regulation of tetrapyrrole catabolic process [GO:1901404], regulation of toluene catabolic process [GO:1901434], regulation of ferulate catabolic process [GO:1901466], regulation of syringal lignin catabolic process [GO:1901469], regulation of gamma-aminobutyric acid catabolic process [GO:1901715], regulation of tRNA catabolic process [GO:1902370], regulation of rRNA catabolic process [GO:1902374], regulation of ornithine catabolic process [GO:1903266], regulation of DNA catabolic process [GO:1903624], regulation of ubiquitin-dependent protein catabolic process [GO:2000058], GO:2000295, regulation of miRNA catabolic process [GO:2000625], regulation of receptor catabolic process [GO:2000644], regulation of amylopectin catabolic process [GO:2000945], regulation of L-proline catabolic process to L-glutamate [GO:2001156] Relationships: is a type of regulation of metabolic process [GO:0019222]; regulates catabolic process [GO:0009056]